melanocyte adhesion [GO:0097326] (biological process) References: PMID:22637532 Sources: CL:0000148, GOC:uh Relationships: is a type of epithelial cell-cell adhesion [GO:0090136] Definition: The attachment of a melanocyte to another cell via adhesion molecules.